connective tissue replacement [GO:0097709] (biological process) Relationships: is a type of tissue remodeling [GO:0048771] References: PMID:25590961 Sources: GOC:BHF, GOC:BHF_miRNA, GOC:bc Subtypes: connective tissue replacement involved in inflammatory response wound healing [GO:0002248] Regulation: regulated by regulation of connective tissue replacement [GO:1905203]; negatively regulated by negative regulation of connective tissue replacement [GO:1905204]; positively regulated by positive regulation of connective tissue replacement [GO:1905205] Definition: The series of events leading to growth of connective tissue when loss of tissues that are incapable of regeneration occurs, or when fibrinous exudate cannot be adequately cleared.